beak formation [GO:0071730] (BP) Relationships: is a type of anatomical structure formation involved in morphogenesis [GO:0048646]; BFO_0000050 beak morphogenesis [GO:0071729] Definition: The process that gives rise to the beak. This process pertains to the initial formation of a structure from unspecified parts. The avian beak is an external anatomical structure, in the head region, that is adapted for feeding self and young, catching prey, probing, etc. It encompasses, but is not restricted to, the maxilla, mandible, maxillary rhamphotheca, mandibular rhamphotheca, nostril, nasal fossa, nasal bones, egg tooth and rictus. Sources: GOC:lp, ISBN:0702008729